{
  "gene_symbol": "RYK",
  "gene_name": "Tyrosine-protein kinase RYK",
  "gene": "UniProtKB:P34925",
  "term_id": "GO:0007169",
  "term_label": "cell surface receptor protein tyrosine kinase signaling pathway"
}